response to type II interferon [GO:0034341] (biological process) Also known as: response to interferon-gamma, response to type II IFN, response to immune interferon, response to gamma-interferon Relationships: is a type of response to cytokine [GO:0034097]; is part of innate immune response [GO:0045087] Definition: Any process that results in a change in state or activity of a cell or an organism (in terms of movement, secretion, enzyme production, gene expression, etc.) as a result of an interferon-gamma stimulus. Interferon-gamma is also known as type II interferon. References: PMID:15546383 Sources: GOC:add, ISBN:0126896631 Subtypes: cellular response to type II interferon [GO:0071346] Regulation: regulated by regulation of response to type II interferon [GO:0060330]; RO_0002212 by GO:0060331; positively regulated by positive regulation of response to type II interferon [GO:0060332]